{
  "term_id": "GO:0016020",
  "gene": "UniProtKB:Q6J4K2",
  "term_label": "membrane",
  "gene_name": "Mitochondrial sodium_calcium exchanger protein",
  "gene_symbol": "SLC8B1"
}